{
  "gene_name": "Protein FAM78A",
  "term_label": "Unknown cellular component",
  "gene_symbol": "FAM78A",
  "term_id": "UNKNOWN:0003",
  "gene": "UniProtKB:Q5JUQ0"
}